{
  "gene_symbol": "GDA",
  "gene": "UniProtKB:Q9Y2T3",
  "term_id": "GO:0008270",
  "term_label": "zinc ion binding",
  "gene_name": "Guanine deaminase"
}